venom-mediated suppression of fibrinolysis [GO:0140099] (BP) Relationships: is a type of venom-mediated perturbation of hemostasis [GO:0044483] References: PMID:19236611, PMID:22359676, PMID:27208884, PMID:35716829 Definition: A process in which an organism inhibits or disrupts fibrinolysis in another organism via the action of a venom. Fibrinolysis is the solubilization of fibrin in the bloodstream. Anti-fibrinolytic proteins reduce bleeding at the bite or sting site of the prey. Also known as: envenomation suppressing fibrinolysis in another organism